{
  "gene": "UniProtKB:Q92692",
  "gene_name": "Nectin-2",
  "gene_symbol": "NECTIN2",
  "term_label": "apical junction complex",
  "term_id": "GO:0043296"
}